{
  "gene_name": "Probable G-protein coupled receptor 33",
  "gene_symbol": "GPR33",
  "gene": "UniProtKB:Q49SQ1",
  "term_id": "GO:0006954",
  "term_label": "inflammatory response"
}